{
  "gene_name": "Importin subunit alpha-1",
  "term_label": "nuclear localization sequence binding",
  "term_id": "GO:0008139",
  "gene_symbol": "KPNA2",
  "gene": "UniProtKB:P52292"
}